{
  "gene_name": "E3 ubiquitin-protein ligase MARCHF2",
  "term_id": "UNKNOWN:0003",
  "gene_symbol": "MARCHF2",
  "gene": "UniProtKB:Q9P0N8",
  "term_label": "Unknown cellular component"
}